{
  "term_id": "GO:0005737",
  "gene_symbol": "APOBEC3F",
  "gene_name": "DNA dC-dU-editing enzyme APOBEC-3F",
  "gene": "UniProtKB:Q8IUX4",
  "term_label": "cytoplasm"
}